{
  "gene_name": "Period circadian protein homolog 2",
  "gene": "UniProtKB:O15055",
  "term_label": "negative regulation of transcription by RNA polymerase II",
  "term_id": "GO:0000122",
  "gene_symbol": "PER2"
}